{
  "gene_symbol": "FBXO21",
  "term_id": "UNKNOWN:0001",
  "gene": "UniProtKB:O94952",
  "gene_name": "F-box only protein 21",
  "term_label": "Unknown molecular function"
}